{
  "gene": "UniProtKB:P08571",
  "gene_symbol": "CD14",
  "term_label": "toll-like receptor 4 signaling pathway",
  "term_id": "GO:0034142",
  "gene_name": "Monocyte differentiation antigen CD14"
}